{
  "gene": "UniProtKB:Q9HBD1",
  "gene_symbol": "RC3H2",
  "term_id": "GO:0003725",
  "gene_name": "Roquin-2",
  "term_label": "double-stranded RNA binding"
}